{
  "term_label": "Unknown biological process",
  "gene_symbol": "ZYG11A",
  "gene": "UniProtKB:Q6WRX3",
  "term_id": "UNKNOWN:0002",
  "gene_name": "Protein zyg-11 homolog A"
}